negative regulation of oligopeptide transport [GO:2000877] (biological process) Subtypes: negative regulation of dipeptide transport [GO:2000879] Definition: Any process that stops, prevents or reduces the frequency, rate or extent of oligopeptide transport. Sources: GOC:obol Relationships: is a type of negative regulation of transport [GO:0051051]; is a type of regulation of oligopeptide transport [GO:0090088]; RO_0002212 oligopeptide transport [GO:0006857]